{
  "gene_name": "Homeobox protein PKNOX2",
  "gene_symbol": "PKNOX2",
  "term_label": "DNA-binding transcription factor activity",
  "term_id": "GO:0003700",
  "gene": "UniProtKB:Q96KN3"
}